{
  "gene_name": "Carbohydrate sulfotransferase 6",
  "gene": "UniProtKB:Q9GZX3",
  "gene_symbol": "CHST6",
  "term_label": "trans-Golgi network",
  "term_id": "GO:0005802"
}